basement membrane disassembly [GO:0034769] (biological process) References: PMID:17301221 Sources: GOC:sart Also known as: basal lamina disassembly Relationships: is a type of extracellular matrix disassembly [GO:0022617]; is a type of basement membrane organization [GO:0071711] Subtypes: basement membrane disassembly involved in semicircular canal fusion [GO:0060882] Note: Note that this term has no relationship to 'membrane disassembly ; GO:0030397' because the basement membrane is not a lipid bilayer. Definition: The controlled breakdown of the basement membrane in the context of a normal process such as imaginal disc eversion.